{
  "gene_symbol": "MYZAP",
  "term_id": "GO:0005665",
  "term_label": "RNA polymerase II, core complex",
  "gene": "UniProtKB:P0CAP1",
  "gene_name": "Myocardial zonula adherens protein"
}